{
  "term_label": "SRP-dependent cotranslational protein targeting to membrane, translocation",
  "gene": "UniProtKB:P60468",
  "gene_name": "Protein transport protein Sec61 subunit beta",
  "gene_symbol": "SEC61B",
  "term_id": "GO:0006616"
}